cyanophycin synthetase activity (L-arginine-adding) [GO:0071161] (molecular function) Definition: Catalysis of the reaction: ATP + [L-Asp(4-L-Arg)]n-L-Asp + L-arginine = ADP + phosphate + [L-Asp(4-L-Arg)]n+1. Sources: EC:6.3.2.30 Relationships: is a type of cyanophycin synthetase activity [GO:0043860]